{
  "term_id": "GO:0005549",
  "term_label": "odorant binding",
  "gene_symbol": "OR5T1",
  "gene": "UniProtKB:Q8NG75",
  "gene_name": "Olfactory receptor 5T1"
}